{
  "gene": "UniProtKB:Q96RI1",
  "term_label": "RNA polymerase II cis-regulatory region sequence-specific DNA binding",
  "term_id": "GO:0000978",
  "gene_name": "Bile acid receptor",
  "gene_symbol": "NR1H4"
}